monolayer-surrounded lipid storage body [GO:0012511] (cellular component) Sources: GOC:mtg_sensu, ISBN:0943088372 Also known as: oil body, oilbody, oleosome, spherosome Definition: A subcellular organelle of plant cells surrounded by 'half-unit' or a monolayer membrane instead of the more usual bilayer. The storage body has a droplet of triglyceride surrounded by a monolayer of phospholipids, interacting with the triglycerides and the hydrophilic head groups facing the cytosol, and containing major protein components called oleosins. Relationships: is a type of lipid droplet [GO:0005811]